selenol Se-methyltransferase activity [GO:0098603] (molecular function) Relationships: is a type of GO:0008168 Definition: Catalysis of the reaction: R + Se-Adenosylselenomethionine = CH3-R + Se-Adenosyl-L-selenohomocysteine. References: PMID:1711890